{
  "gene_name": "Transcriptional enhancer factor TEF-3",
  "term_label": "DNA-binding transcription factor activity, RNA polymerase II-specific",
  "term_id": "GO:0000981",
  "gene_symbol": "TEAD4",
  "gene": "UniProtKB:Q15561"
}